{
  "gene_name": "DNA topoisomerase 3-alpha",
  "term_id": "GO:0031422",
  "gene": "UniProtKB:Q13472",
  "term_label": "RecQ family helicase-topoisomerase III complex",
  "gene_symbol": "TOP3A"
}